regulation of meristem structural organization [GO:0009934] (biological process) Relationships: is a type of GO:0050793; regulates meristem structural organization [GO:0009933] Sources: GOC:jid Definition: Any process that modulates the frequency, rate or extent of meristem organization. Also known as: regulation of meristem organization, regulation of meristem organisation